{
  "gene_name": "Piwi-like protein 1",
  "gene": "UniProtKB:Q96J94",
  "term_label": "P granule",
  "gene_symbol": "PIWIL1",
  "term_id": "GO:0043186"
}